{
  "gene_symbol": "KCNE3",
  "term_id": "GO:0044325",
  "gene_name": "Potassium voltage-gated channel subfamily E member 3",
  "gene": "UniProtKB:Q9Y6H6",
  "term_label": "transmembrane transporter binding"
}